{
  "gene_name": "Complement component receptor 1-like protein",
  "gene": "UniProtKB:Q2VPA4",
  "gene_symbol": "CR1L",
  "term_label": "negative regulation of complement activation, classical pathway",
  "term_id": "GO:0045959"
}